{
  "term_id": "GO:0004674",
  "gene": "UniProtKB:Q96SB4",
  "term_label": "protein serine/threonine kinase activity",
  "gene_symbol": "SRPK1",
  "gene_name": "SRSF protein kinase 1"
}